negative regulation of protein localization to membrane [GO:1905476] (biological process) References: PMID:26911690 Sources: GOC:PARL, GOC:TermGenie, GOC:bc, GO_REF:0000058 Definition: Any process that stops, prevents or reduces the frequency, rate or extent of protein localization to membrane. Relationships: is a type of negative regulation of cellular process [GO:0048523]; is_a negative regulation of protein localization [GO:1903828]; is_a GO:1905475; negatively regulates protein localization to membrane [GO:0072657] Subtypes: negative regulation of protein targeting to vacuolar membrane [GO:1900484], GO:1903077, negative regulation of protein localization to ciliary membrane [GO:1903568], GO:1903910, negative regulation of t-SNARE clustering [GO:1904033], negative regulation of protein localization to basolateral plasma membrane [GO:1904509] Also known as: down regulation of protein localisation in membrane, down regulation of protein localization in membrane, down regulation of protein localization to membrane, down-regulation of protein localisation in membrane, down-regulation of protein localization in membrane, down-regulation of protein localization to membrane, downregulation of protein localisation in membrane, downregulation of protein localization in membrane, downregulation of protein localization to membrane, negative regulation of protein localisation in membrane, negative regulation of protein localization in membrane, inhibition of protein localisation in membrane, inhibition of protein localization in membrane, inhibition of protein localization to membrane